{
  "gene_symbol": "HACD1",
  "term_id": "GO:0018812",
  "gene_name": "Very-long-chain (3R)-3-hydroxyacyl-CoA dehydratase 1",
  "gene": "UniProtKB:B0YJ81",
  "term_label": "3-hydroxyacyl-CoA dehydratase activity"
}